mesonephric glomerular parietal epithelial cell differentiation [GO:0061253] (biological process) Definition: The process in which a relatively unspecialized cell acquires specialized features of a mesonephric glomerular parietal epithelial cell. Mesonephric glomerular parietal epithelial cells are specialized epithelial cells that form tight junctions as a barrier to protein transport. Sources: GOC:mtg_kidney_jan10 Relationships: is a type of mesonephric glomerular epithelial cell differentiation [GO:0061250]; is a type of glomerular parietal epithelial cell differentiation [GO:0072139]